{
  "term_label": "ephrin receptor signaling pathway",
  "term_id": "GO:0048013",
  "gene_symbol": "EPHB1",
  "gene_name": "Ephrin type-B receptor 1",
  "gene": "UniProtKB:P54762"
}